{
  "term_id": "GO:0042307",
  "term_label": "positive regulation of protein import into nucleus",
  "gene_name": "Zinc finger protein ZPR1",
  "gene_symbol": "ZPR1",
  "gene": "UniProtKB:O75312"
}